{
  "term_label": "plasma membrane",
  "gene_symbol": "PLXNB1",
  "gene_name": "Plexin-B1",
  "term_id": "GO:0005886",
  "gene": "UniProtKB:O43157"
}